{
  "gene": "UniProtKB:O60749",
  "term_id": "GO:0034498",
  "gene_symbol": "SNX2",
  "gene_name": "Sorting nexin-2",
  "term_label": "early endosome to Golgi transport"
}